{
  "gene": "UniProtKB:Q12846",
  "gene_symbol": "STX4",
  "term_id": "GO:0000149",
  "term_label": "SNARE binding",
  "gene_name": "Syntaxin-4"
}